{
  "gene_name": "Protein Niban 2",
  "term_id": "UNKNOWN:0001",
  "term_label": "Unknown molecular function",
  "gene_symbol": "NIBAN2",
  "gene": "UniProtKB:Q96TA1"
}